{
  "term_label": "cell cortex",
  "gene": "UniProtKB:Q8TEW8",
  "gene_symbol": "PARD3B",
  "gene_name": "Partitioning defective 3 homolog B",
  "term_id": "GO:0005938"
}